{
  "gene": "UniProtKB:O43529",
  "gene_symbol": "CHST10",
  "term_id": "GO:0008146",
  "term_label": "sulfotransferase activity",
  "gene_name": "Carbohydrate sulfotransferase 10"
}